phenyl-phosphate phosphatase/carboxylase activity [GO:0018862] (molecular function) Definition: Catalysis of the reaction: 4-hydroxybenzoate + H+ + phosphate = CO2 + H2O + phenyl phosphate. Relationships: is a type of GO:0016831 Also known as: phenylphosphate carboxylase activity Sources: RHEA:74015